negative regulation of prostaglandin biosynthetic process [GO:0031393] (biological process) Also known as: down regulation of prostaglandin biosynthetic process, down-regulation of prostaglandin biosynthetic process, downregulation of prostaglandin biosynthetic process, negative regulation of prostaglandin anabolism, negative regulation of prostaglandin biosynthesis, negative regulation of prostaglandin formation, negative regulation of prostaglandin synthesis, inhibition of prostaglandin biosynthetic process Sources: GOC:mah Relationships: is_a GO:0031392; is a type of negative regulation of fatty acid biosynthetic process [GO:0045717]; negatively regulates prostaglandin biosynthetic process [GO:0001516] Definition: Any process that stops, prevents, or reduces the frequency, rate or extent of the chemical reactions and pathways resulting in the formation of prostaglandin.